positive regulation of 18-methylnonadec-1-ene biosynthetic process [GO:1900952] (biological process) Definition: Any process that activates or increases the frequency, rate or extent of 18-methylnonadec-1-ene biosynthetic process. Sources: GOC:TermGenie, GOC:mengo_curators Relationships: is_a positive regulation of olefin biosynthetic process [GO:1900913]; is a type of regulation of 18-methylnonadec-1-ene biosynthetic process [GO:1900950]; positively regulates GO:1900881 Also known as: activation of 18-methylnonadec-1-ene anabolism, activation of 18-methylnonadec-1-ene biosynthesis, activation of 18-methylnonadec-1-ene formation, activation of 18-methylnonadec-1-ene synthesis, positive regulation of 18-methylnonadec-1-ene anabolism, positive regulation of 18-methylnonadec-1-ene biosynthesis, positive regulation of 18-methylnonadec-1-ene formation, positive regulation of 18-methylnonadec-1-ene synthesis, up regulation of 18-methylnonadec-1-ene anabolism, up regulation of 18-methylnonadec-1-ene biosynthesis, up regulation of 18-methylnonadec-1-ene biosynthetic process, up regulation of 18-methylnonadec-1-ene formation, up regulation of 18-methylnonadec-1-ene synthesis, up-regulation of 18-methylnonadec-1-ene anabolism, up-regulation of 18-methylnonadec-1-ene biosynthesis, up-regulation of 18-methylnonadec-1-ene biosynthetic process, up-regulation of 18-methylnonadec-1-ene formation, up-regulation of 18-methylnonadec-1-ene synthesis, upregulation of 18-methylnonadec-1-ene anabolism, upregulation of 18-methylnonadec-1-ene biosynthesis, upregulation of 18-methylnonadec-1-ene biosynthetic process, upregulation of 18-methylnonadec-1-ene formation, upregulation of 18-methylnonadec-1-ene synthesis, activation of 18-methylnonadec-1-ene biosynthetic process